{
  "gene_symbol": "OXER1",
  "gene_name": "Oxoeicosanoid receptor 1",
  "gene": "UniProtKB:Q8TDS5",
  "term_label": "G protein-coupled receptor activity",
  "term_id": "GO:0004930"
}